{
  "gene_symbol": "A0A7I2V6D3",
  "term_label": "Unknown molecular function",
  "term_id": "UNKNOWN:0001",
  "gene": "UniProtKB:A0A7I2V6D3",
  "gene_name": "Uncharacterized protein"
}